{
  "gene": "UniProtKB:Q2NL98",
  "term_id": "UNKNOWN:0001",
  "gene_name": "Vimentin-type intermediate filament-associated coiled-coil protein",
  "term_label": "Unknown molecular function",
  "gene_symbol": "VMAC"
}